oculomotor nerve maturation [GO:0021625] (biological process) Relationships: is a type of cranial nerve maturation [GO:0021605]; is part of GO:0021557 Sources: GOC:cls, GOC:dgh, GOC:dph, GOC:jid, GO_REF:0000021 Definition: A developmental process, independent of morphogenetic (shape) change, that is required for the oculomotor nerve to attain its fully functional state. This motor nerve innervates all extraocular muscles except the superior oblique and the lateral rectus muscles. The superior division supplies the levator palpebrae superioris and superior rectus muscles. The inferior division supplies the medial rectus, inferior rectus and inferior oblique muscles. This nerve also innervates the striated muscles of the eyelid. Pupillary constriction and lens movement are mediated by this nerve for near vision. In the orbit the inferior division sends branches that enter the ciliary ganglion where they form functional contacts (synapses) with the ganglion cells. The ganglion cells send nerve fibers into the back of the eye where they travel to ultimately innervate the ciliary muscle and the constrictor pupillae muscle. Also known as: CN III maturation